{
  "term_label": "external side of plasma membrane",
  "gene_symbol": "MS4A1",
  "gene": "UniProtKB:P11836",
  "term_id": "GO:0009897",
  "gene_name": "B-lymphocyte antigen CD20"
}